{
  "term_label": "cytoplasm",
  "gene_symbol": "PRPSAP2",
  "term_id": "GO:0005737",
  "gene": "UniProtKB:O60256",
  "gene_name": "Phosphoribosyl pyrophosphate synthase-associated protein 2"
}